{
  "term_id": "UNKNOWN:0001",
  "term_label": "Unknown molecular function",
  "gene": "UniProtKB:Q5T7P2",
  "gene_symbol": "LCE1A",
  "gene_name": "Late cornified envelope protein 1A"
}